collagen beaded filament [GO:0098647] (cellular component) References: PMID:19693541 Sources: GOC:dos Also known as: beads on a string Relationships: is a type of complex of collagen trimers [GO:0098644]; is a type of GO:0099512; is part of basement membrane/interstitial matrix interface [GO:0140086] Definition: A supramolecular assembly of collagen trimers with a 'beads on a string'-like structure.